rRNA (cytosine-N4-)-methyltransferase activity [GO:0071424] (molecular function) Definition: Catalysis of the reaction: a cytidine in rRNA + S-adenosyl-L-methionine = an N(4)-methylcytidine in rRNA + H+ + S-adenosyl-L-homocysteine. References: PMID:19965768 Sources: GOC:imk, RHEA:62520 Relationships: is a type of GO:0008170; is a type of GO:0016434